{
  "term_id": "UNKNOWN:0001",
  "gene": "UniProtKB:A0A0C4DH68",
  "gene_name": "Immunoglobulin kappa variable 2-24",
  "gene_symbol": "IGKV2-24",
  "term_label": "Unknown molecular function"
}